{
  "gene_symbol": "VPS53",
  "term_id": "GO:0000938",
  "term_label": "GARP complex",
  "gene": "UniProtKB:Q5VIR6",
  "gene_name": "Vacuolar protein sorting-associated protein 53 homolog"
}